{
  "term_label": "D-ribulose-phosphate 3-epimerase activity",
  "gene": "UniProtKB:Q96AT9",
  "term_id": "GO:0004750",
  "gene_symbol": "RPE",
  "gene_name": "Ribulose-phosphate 3-epimerase"
}